{
  "gene_name": "S100P-binding protein",
  "gene": "UniProtKB:Q96BU1",
  "term_label": "calcium-dependent protein binding",
  "term_id": "GO:0048306",
  "gene_symbol": "S100PBP"
}